{
  "gene_name": "Guanine nucleotide-binding protein-like 3-like protein",
  "gene": "UniProtKB:Q9NVN8",
  "term_id": "UNKNOWN:0001",
  "term_label": "Unknown molecular function",
  "gene_symbol": "GNL3L"
}